{
  "gene": "UniProtKB:Q17RY6",
  "gene_symbol": "LY6K",
  "gene_name": "Lymphocyte antigen 6K",
  "term_id": "GO:0007339",
  "term_label": "binding of sperm to zona pellucida"
}